{
  "gene": "UniProtKB:P13284",
  "gene_name": "Gamma-interferon-inducible lysosomal thiol reductase",
  "term_label": "lysosome",
  "gene_symbol": "IFI30",
  "term_id": "GO:0005764"
}